{
  "gene_name": "Adhesion G protein-coupled receptor L3",
  "gene_symbol": "ADGRL3",
  "gene": "UniProtKB:Q9HAR2",
  "term_label": "G protein-coupled receptor activity",
  "term_id": "GO:0004930"
}